{
  "gene_name": "Olfactory receptor 51V1",
  "gene_symbol": "OR51V1",
  "term_id": "GO:0005886",
  "term_label": "plasma membrane",
  "gene": "UniProtKB:Q9H2C8"
}